{
  "term_id": "GO:0005634",
  "gene_symbol": "FAM53A",
  "gene": "UniProtKB:Q6NSI3",
  "term_label": "nucleus",
  "gene_name": "Protein FAM53A"
}